{
  "gene_name": "Olfactory receptor 2A4",
  "term_id": "GO:0004984",
  "gene": "UniProtKB:O95047",
  "term_label": "olfactory receptor activity",
  "gene_symbol": "OR2A4"
}